{
  "gene_symbol": "PTGIR",
  "gene": "UniProtKB:P43119",
  "term_id": "GO:0016501",
  "term_label": "prostacyclin receptor activity",
  "gene_name": "Prostacyclin receptor"
}